RNA localization to chromatin [GO:1990280] (biological process) References: PMID:22582262 Sources: GOC:dos, GOC:mah Relationships: is a type of RNA localization [GO:0006403] Definition: A process in which RNA is transported to and maintained in a part of a chromosome that is organized into chromatin. Also known as: RNA localisation to chromatin